{
  "term_label": "cytokine-mediated signaling pathway",
  "term_id": "GO:0019221",
  "gene_symbol": "CSF2RA",
  "gene_name": "Granulocyte-macrophage colony-stimulating factor receptor subunit alpha",
  "gene": "UniProtKB:P15509"
}